{
  "term_id": "GO:0005886",
  "term_label": "plasma membrane",
  "gene_name": "Solute carrier family 41 member 3",
  "gene_symbol": "SLC41A3",
  "gene": "UniProtKB:Q96GZ6"
}